{
  "term_id": "GO:0006886",
  "gene_name": "Ras-related protein Rab-43",
  "gene": "UniProtKB:Q86YS6",
  "gene_symbol": "RAB43",
  "term_label": "intracellular protein transport"
}